regulation of lipoprotein particle clearance [GO:0010984] (BP) Definition: Any process that modulates the rate, frequency, or extent of lipoprotein particle clearance. Lipoprotein particle clearance is the process in which a lipoprotein particle is removed from the blood via receptor-mediated endocytosis and its constituent parts degraded. Sources: GOC:BHF, GOC:dph, GOC:tb Subtypes: regulation of very-low-density lipoprotein particle clearance [GO:0010915], GO:0010982, negative regulation of lipoprotein particle clearance [GO:0010985], positive regulation of lipoprotein particle clearance [GO:0010986], regulation of low-density lipoprotein particle clearance [GO:0010988], GO:0090320 Relationships: is a type of regulation of multicellular organismal process [GO:0051239]; regulates plasma lipoprotein particle clearance [GO:0034381]